{
  "gene": "UniProtKB:P54652",
  "term_id": "GO:0005886",
  "gene_name": "Heat shock-related 70 kDa protein 2",
  "term_label": "plasma membrane",
  "gene_symbol": "HSPA2"
}